{
  "gene_symbol": "PDZD8",
  "term_label": "mitochondria-associated endoplasmic reticulum membrane contact site",
  "term_id": "GO:0044233",
  "gene": "UniProtKB:Q8NEN9",
  "gene_name": "PDZ domain-containing protein 8"
}